{
  "term_id": "UNKNOWN:0001",
  "gene_name": "Stannin",
  "gene": "UniProtKB:O75324",
  "term_label": "Unknown molecular function",
  "gene_symbol": "SNN"
}